{
  "gene_symbol": "VPS26B",
  "term_label": "retrograde transport, endosome to Golgi",
  "gene": "UniProtKB:Q4G0F5",
  "term_id": "GO:0042147",
  "gene_name": "Vacuolar protein sorting-associated protein 26B"
}